microvillus assembly [GO:0030033] (biological process) Definition: Formation of a microvillus, a thin cylindrical membrane-covered projection on the surface of a cell. Sources: GOC:mah, ISBN:0815316194 Relationships: is a type of microvillus organization [GO:0032528]; is a type of plasma membrane bounded cell projection assembly [GO:0120031] Also known as: microvillus biogenesis Regulation: regulated by GO:0032534; RO_0002212 by GO:1903697; positively regulated by positive regulation of microvillus assembly [GO:1903698]